isopropanol dehydrogenase (NADP+) activity [GO:0050009] (molecular function) Definition: Catalysis of the reaction: NADP+ + propan-2-ol = acetone + H+ + NADPH. Relationships: is a type of GO:0016616 Also known as: propan-2-ol:NADP+ oxidoreductase activity Sources: EC:1.1.1.80, RHEA:21792